{
  "gene_name": "Secretogranin-3",
  "gene_symbol": "SCG3",
  "gene": "UniProtKB:Q8WXD2",
  "term_id": "UNKNOWN:0001",
  "term_label": "Unknown molecular function"
}